{
  "gene": "UniProtKB:Q96I99",
  "term_id": "GO:0004776",
  "gene_symbol": "SUCLG2",
  "gene_name": "Succinate--CoA ligase [GDP-forming] subunit beta, mitochondrial",
  "term_label": "succinate-CoA ligase (GDP-forming) activity"
}